heparan sulfate proteoglycan biosynthetic process [GO:0015012] (biological process) Relationships: is a type of proteoglycan biosynthetic process [GO:0030166]; is a type of GO:0030201; is a type of protein O-linked glycosylation via xylose [GO:0180064] Definition: The chemical reactions and pathways resulting in the formation of heparan sulfate proteoglycans, which consist of a core protein linked to a heparan sulfate glycosaminoglycan. The heparan sulfate chain is composed of the repeating disaccharide unit beta-(1,4)-N-acetyl-D-glucosamine-alpha-(1,4)-hexuronic acid, the former being either sulfated or deacetylated on its amino group as well as sulfated on one of its hydroxyl groups, and the latter being e a mixture of sulfated and nonsulfated D-glucuronic and L-iduronic acids. Heparan sulfate chains are covalently linked to serine/threonine residues (O-linked) of the core protein via a tetrasaccharide linker sequence (xylose-galactose-galactose-glucuronate). Also known as: heparan sulfate proteoglycan anabolism, heparan sulfate proteoglycan biosynthesis, heparan sulfate proteoglycan formation, heparan sulfate proteoglycan synthesis, heparan sulphate proteoglycan biosynthesis, heparan sulphate proteoglycan biosynthetic process, heparin proteoglycan biosynthetic process Regulation: regulated by regulation of heparan sulfate proteoglycan biosynthetic process [GO:0010908]; positively regulated by positive regulation of heparan sulfate proteoglycan biosynthetic process [GO:0010909] References: PMID:27241222